positive regulation of peptidoglycan recognition protein signaling pathway [GO:0061059] (biological process) Sources: GOC:dph Relationships: is a type of regulation of peptidoglycan recognition protein signaling pathway [GO:0061058]; is a type of positive regulation of pattern recognition receptor signaling pathway [GO:0062208]; is a type of positive regulation of defense response to bacterium [GO:1900426]; positively regulates peptidoglycan recognition protein signaling pathway [GO:0061057] Also known as: positive regulation of peptidoglycan recognition protein signalling pathway Definition: Any process that increases the rate, frequency, or extent of the peptidoglycan recognition protein signaling pathway.